regulation of chromosome condensation [GO:0060623] (biological process) Definition: Any process that modulates the rate, frequency, or extent of chromosome condensation, the progressive compaction of dispersed interphase chromatin into threadlike chromosomes prior to mitotic or meiotic nuclear division, or during apoptosis, in eukaryotic cells. Subtypes: negative regulation of chromosome condensation [GO:1902340], regulation of mitotic chromosome condensation [GO:1903379], positive regulation of chromosome condensation [GO:1905821] Sources: GOC:dph, GOC:tb Relationships: is a type of regulation of chromosome organization [GO:0033044]; RO_0002211 GO:0030261